{
  "gene": "UniProtKB:Q9H2M9",
  "term_id": "GO:0042734",
  "gene_symbol": "RAB3GAP2",
  "term_label": "presynaptic membrane",
  "gene_name": "Rab3 GTPase-activating protein non-catalytic subunit"
}